{
  "term_id": "GO:0003730",
  "gene": "UniProtKB:Q9Y534",
  "term_label": "mRNA 3'-UTR binding",
  "gene_symbol": "CSDC2",
  "gene_name": "Cold shock domain-containing protein C2"
}